glial cell projection [GO:0097386] (cellular component) Definition: A prolongation or process extending from a glial cell. Also known as: glial process, glial projection Sources: GOC:mc Relationships: is a type of GO:0120025 Subtypes: capitate projection [GO:0097387], astrocyte projection [GO:0097449], GO:0097454, GO:0097455, terminal loop [GO:0097456]